{
  "gene_symbol": "SETBP1",
  "gene_name": "SET-binding protein",
  "term_label": "histone H3K4 methyltransferase activity",
  "term_id": "GO:0042800",
  "gene": "UniProtKB:Q9Y6X0"
}